{
  "term_label": "cell morphogenesis",
  "term_id": "GO:0000902",
  "gene": "UniProtKB:P33151",
  "gene_symbol": "CDH5",
  "gene_name": "Cadherin-5"
}